{
  "term_id": "GO:0017147",
  "gene_symbol": "FZD6",
  "gene_name": "Frizzled-6",
  "gene": "UniProtKB:O60353",
  "term_label": "Wnt-protein binding"
}